{
  "term_id": "UNKNOWN:0002",
  "gene_symbol": "MFSD3",
  "gene": "UniProtKB:Q96ES6",
  "gene_name": "Major facilitator superfamily domain-containing protein 3",
  "term_label": "Unknown biological process"
}